regulation of R7 cell fate commitment [GO:0106396] (biological process) Definition: Any process that modulates the frequency, rate or extent of R7 cell fate commitment. References: PMID:22878552 Sources: GOC:ha Subtypes: GO:0106397, negative regulation of R7 cell fate commitment [GO:0106398] Relationships: is a type of GO:0010453; regulates R7 cell fate commitment [GO:0007465]